protein localization to condensed nuclear chromosome [GO:1903084] (biological process) Definition: A process in which a protein is transported to, or maintained in, a location within a condensed nuclear chromosome. References: PMID:12707312 Sources: GOC:TermGenie, GOC:kmv, GO_REF:0000087 Also known as: protein localisation in condensed nuclear chromosome, protein localisation to condensed nuclear chromosome, protein localization in condensed nuclear chromosome Relationships: is a type of protein localization to nucleus [GO:0034504]; is a type of protein localization to condensed chromosome [GO:1903083] Subtypes: protein localization to linear element [GO:0036181]